anaerobic catabolism of pairs of amino acids [GO:0019668] (biological process) Also known as: cofermentation of pairs of amino acids, Stickland reaction Definition: The anaerobic chemical reactions and pathways resulting in the breakdown of amino acids; in these reactions, one amino acid is oxidised (acts as an electron donor) and a different amino acid is reduced (acts as an electron acceptor); oxidation of the electron-donating amino acid yields energy in the form of ATP. References: PMID:13140081 Sources: GOC:mah Relationships: is a type of anaerobic amino acid catabolic process [GO:0019665]